{
  "gene_name": "E3 ubiquitin-protein ligase RNF186",
  "term_id": "GO:0043161",
  "gene_symbol": "RNF186",
  "gene": "UniProtKB:Q9NXI6",
  "term_label": "proteasome-mediated ubiquitin-dependent protein catabolic process"
}